protein localization to somatodendritic compartment [GO:0061938] (biological process) References: PMID:18341993 Also known as: somatodendritic protein localization Definition: A process in which a protein is transported to or maintained in a location within the somatodendritic compartment. Relationships: is a type of intracellular protein localization [GO:0008104]